{
  "gene_name": "U3 small nucleolar RNA-associated protein 6 homolog",
  "term_label": "maturation of SSU-rRNA from tricistronic rRNA transcript (SSU-rRNA, 5.8S rRNA, LSU-rRNA)",
  "gene": "UniProtKB:Q9NYH9",
  "gene_symbol": "UTP6",
  "term_id": "GO:0000462"
}